{
  "gene": "UniProtKB:Q9NVK5",
  "gene_name": "FGFR1 oncogene partner 2",
  "term_label": "Unknown molecular function",
  "gene_symbol": "FGFR1OP2",
  "term_id": "UNKNOWN:0001"
}